{
  "term_label": "actin polymerization or depolymerization",
  "gene_symbol": "FLII",
  "term_id": "GO:0008154",
  "gene_name": "Protein flightless-1 homolog",
  "gene": "UniProtKB:Q13045"
}